{
  "gene_symbol": "TNFSF10",
  "gene": "UniProtKB:P50591",
  "term_id": "GO:2001238",
  "gene_name": "Tumor necrosis factor ligand superfamily member 10",
  "term_label": "positive regulation of extrinsic apoptotic signaling pathway"
}